{
  "term_label": "Unknown molecular function",
  "gene": "UniProtKB:Q9H7S9",
  "gene_symbol": "ZNF703",
  "term_id": "UNKNOWN:0001",
  "gene_name": "Zinc finger protein 703"
}